{
  "gene": "UniProtKB:P02656",
  "term_id": "GO:0010897",
  "gene_symbol": "APOC3",
  "term_label": "negative regulation of triglyceride catabolic process",
  "gene_name": "Apolipoprotein C-III"
}